{
  "gene_symbol": "HRG",
  "term_id": "GO:0008201",
  "gene_name": "Histidine-rich glycoprotein",
  "gene": "UniProtKB:P04196",
  "term_label": "heparin binding"
}